myoblast development [GO:0048627] (biological process) Relationships: is a type of GO:0048468; is part of myoblast differentiation [GO:0045445] Definition: The process whose specific outcome is the progression of the myoblast over time, from its formation to the mature structure. A myoblast is a mononucleate cell type that, by fusion with other myoblasts, gives rise to the myotubes that eventually develop into skeletal muscle fibers. Sources: CL:0000056, GOC:dph, GOC:mtg_muscle